{
  "gene_name": "Fibroblast growth factor 21",
  "gene": "UniProtKB:Q9NSA1",
  "term_label": "fibroblast growth factor receptor binding",
  "term_id": "GO:0005104",
  "gene_symbol": "FGF21"
}